{
  "gene_name": "Insulin-induced gene 2 protein",
  "gene_symbol": "INSIG2",
  "gene": "UniProtKB:Q9Y5U4",
  "term_id": "GO:0005783",
  "term_label": "endoplasmic reticulum"
}